{
  "term_label": "rod photoreceptor outer segment",
  "gene_name": "Spermatogenesis-associated protein 7",
  "term_id": "GO:0120200",
  "gene": "UniProtKB:Q9P0W8",
  "gene_symbol": "SPATA7"
}